{
  "term_id": "GO:0008569",
  "gene_symbol": "DNAH6",
  "gene": "UniProtKB:Q9C0G6",
  "term_label": "minus-end-directed microtubule motor activity",
  "gene_name": "Dynein axonemal heavy chain 6"
}